leukotriene transport [GO:0071716] (biological process) Subtypes: GO:0071719 Definition: The directed movement of leukotrienes into, out of or within a cell, or between cells, by means of some agent such as a transporter or pore. Leukotrienes are linear C20 endogenous metabolites of arachidonic acid (icosa-5,8,11,14-tetraenoic acid) containing a terminal carboxy function and four or more double bonds (three or more of which are conjugated) as well as other functional groups. Relationships: is a type of icosanoid transport [GO:0071715] Sources: GOC:mah